{
  "gene": "UniProtKB:Q92696",
  "gene_name": "Geranylgeranyl transferase type-2 subunit alpha",
  "term_label": "endoplasmic reticulum to Golgi vesicle-mediated transport",
  "term_id": "GO:0006888",
  "gene_symbol": "RABGGTA"
}